{
  "gene_name": "Mast_stem cell growth factor receptor Kit",
  "term_label": "receptor complex",
  "gene": "UniProtKB:P10721",
  "gene_symbol": "KIT",
  "term_id": "GO:0043235"
}